cell wall modification involved in abscission [GO:0009830] (biological process) Sources: GOC:dph, GOC:lr, GOC:sdb_2009, GOC:tb Definition: A cellular process that results in the breakdown of the cell wall that contributes to the process of abscission. Subtypes: cell wall disassembly involved in floral organ abscission [GO:0060870], plant-type cell wall loosening involved in abscission [GO:1902088] Also known as: cell wall modification during abscission Relationships: is a type of GO:0009827; is a type of GO:0044277; is part of abscission [GO:0009838]